{
  "gene_symbol": "TRIM46",
  "term_id": "UNKNOWN:0001",
  "term_label": "Unknown molecular function",
  "gene_name": "Tripartite motif-containing protein 46",
  "gene": "UniProtKB:Q7Z4K8"
}